{
  "gene_symbol": "SELENON",
  "term_id": "GO:0048741",
  "term_label": "skeletal muscle fiber development",
  "gene": "UniProtKB:Q9NZV5",
  "gene_name": "Selenoprotein N"
}